{
  "term_label": "Unknown biological process",
  "gene": "UniProtKB:P05814",
  "term_id": "UNKNOWN:0002",
  "gene_name": "Beta-casein",
  "gene_symbol": "CSN2"
}